regulation of pigmentation [GO:0120305] (biological process) Relationships: is a type of regulation of biological process [GO:0050789]; regulates GO:0043473 Subtypes: regulation of developmental pigmentation [GO:0048070], background adaptation [GO:0120302] Definition: Any process that modulates the frequency, rate or extent of the deposition or modulates the distribution of coloring matter in an organism. Sources: GOC:krc